{
  "term_label": "GATOR1 complex",
  "term_id": "GO:1990130",
  "gene_symbol": "NPRL3",
  "gene_name": "GATOR complex protein NPRL3",
  "gene": "UniProtKB:Q12980"
}